{
  "gene_name": "Rho-related GTP-binding protein RhoU",
  "term_label": "plasma membrane",
  "gene": "UniProtKB:Q7L0Q8",
  "gene_symbol": "RHOU",
  "term_id": "GO:0005886"
}